{
  "term_id": "GO:0005737",
  "gene_name": "Embryonic polyadenylate-binding protein 2",
  "gene_symbol": "PABPN1L",
  "gene": "UniProtKB:A6NDY0",
  "term_label": "cytoplasm"
}